aluminum ion transmembrane transporter activity [GO:0015083] (molecular function) Relationships: is a type of GO:0022857; is part of GO:1902602 Sources: GOC:ai, GOC:mtg_transport, ISBN:0815340729 Definition: Enables the transfer of aluminum (Al) ions from one side of a membrane to the other. Also known as: aluminium ion transporter activity, aluminium resistance permease activity, aluminum resistance permease activity